heart wedging [GO:0003297] (biological process) Definition: The morphogenetic process in which the aorta inserts between the atrioventricular valves, contributing to the shaping of the heart. Relationships: is a type of anatomical structure morphogenesis [GO:0009653]; is part of GO:0003007 Sources: GOC:mtg_heart